{
  "gene_name": "Cyclin-dependent kinase-like 3",
  "term_label": "nucleus",
  "gene_symbol": "CDKL3",
  "gene": "UniProtKB:Q8IVW4",
  "term_id": "GO:0005634"
}